{
  "gene_symbol": "GPR52",
  "gene": "UniProtKB:Q9Y2T5",
  "gene_name": "G-protein coupled receptor 52",
  "term_id": "GO:0008020",
  "term_label": "G protein-coupled photoreceptor activity"
}